{
  "gene_symbol": "MTRF1",
  "term_id": "GO:0005739",
  "term_label": "mitochondrion",
  "gene_name": "Peptide chain release factor 1, mitochondrial",
  "gene": "UniProtKB:O75570"
}